{
  "gene_name": "Proto-oncogene DBL",
  "gene_symbol": "MCF2",
  "gene": "UniProtKB:P10911",
  "term_label": "cytoplasm",
  "term_id": "GO:0005737"
}